{
  "term_id": "GO:0015562",
  "term_label": "efflux transmembrane transporter activity",
  "gene": "UniProtKB:O00476",
  "gene_symbol": "SLC17A3",
  "gene_name": "Sodium-dependent phosphate transport protein 4"
}